piecemeal microautophagy of the nucleus [GO:0034727] (biological process) Also known as: PMN Definition: Degradation of a cell nucleus by microautophagy. Relationships: is a type of microautophagy [GO:0016237]; is a type of nucleophagy [GO:0044804]; has part GO:1905690 References: PMID:18701704 Sources: GOC:autophagy, GOC:jp